{
  "gene_symbol": "SYNJ2",
  "term_id": "GO:0005737",
  "gene_name": "Synaptojanin-2",
  "gene": "UniProtKB:O15056",
  "term_label": "cytoplasm"
}